{
  "gene_name": "KRAB domain-containing protein 1",
  "term_label": "DNA-binding transcription repressor activity, RNA polymerase II-specific",
  "term_id": "GO:0001227",
  "gene": "UniProtKB:C9JBD0",
  "gene_symbol": "KRBOX1"
}